prechordal plate formation [GO:0021501] (biological process) Definition: The formation of the prechordal plate. The prechordal plate is a thickening of the endoderm at the cranial end of the primitive streak formed by the involution of Spemann's organizer cells. The prechordal plate and the notochord induce the formation of the neural plate from the overlying ectodermal cells. Sources: GOC:cls, GOC:dgh, GOC:dph, GOC:jid, GO_REF:0000021 Relationships: is a type of anatomical structure formation involved in morphogenesis [GO:0048646]; is part of nervous system development [GO:0007399]